long-chain (3S)-3-hydroxyacyl-CoA dehydrogenase (NAD+) activity [GO:0016509] (molecular function) Definition: Catalysis of the reaction: a long-chain (3S)-3-hydroxy fatty acyl-CoA + NAD+ = a long-chain 3-oxo-fatty acyl-CoA + H+ + NADH. A long-chain fatty acid has an aliphatic tail containing 13 to 22 carbons. Sources: RHEA:52656 Also known as: long-chain-3-hydroxyacyl-CoA dehydrogenase (NAD+) activity, LCHAD, beta-hydroxyacyl-CoA dehydrogenase activity, long-chain 3-hydroxyacyl coenzyme A dehydrogenase activity, long-chain-(S)-3-hydroxyacyl-CoA:NAD+ oxidoreductase activity Note: While there is not universal consensus on the lengths of short-, medium-, long- and very-long-chain fatty acids, the GO uses the definitions in ChEBI (see CHEBI:26666, CHEBI:59554, CHEBI:15904 and CHEBI:27283). Relationships: is a type of (3S)-3-hydroxyacyl-CoA dehydrogenase (NAD+) activity [GO:0003857]